vascular wound healing [GO:0061042] (biological process) Definition: Blood vessel formation when new vessels emerge from the proliferation of pre-existing blood vessels and contribute to the series of events that restore integrity to damaged vasculature. Regulation: positively regulated by GO:0035470; regulated by regulation of vascular wound healing [GO:0061043]; negatively regulated by negative regulation of vascular wound healing [GO:0061044] Relationships: is a type of GO:0060055 Sources: GOC:BHF, GOC:dph